{
  "gene": "UniProtKB:Q9UJS0",
  "gene_symbol": "SLC25A13",
  "term_label": "aspartate transmembrane transport",
  "gene_name": "Electrogenic aspartate_glutamate antiporter SLC25A13, mitochondrial",
  "term_id": "GO:0015810"
}